{
  "gene": "UniProtKB:O60518",
  "term_id": "GO:0061608",
  "term_label": "nuclear import signal receptor activity",
  "gene_name": "Ran-binding protein 6",
  "gene_symbol": "RANBP6"
}